{
  "gene_symbol": "ACADM",
  "term_label": "cytoplasm",
  "gene": "UniProtKB:P11310",
  "gene_name": "Medium-chain specific acyl-CoA dehydrogenase, mitochondrial",
  "term_id": "GO:0005737"
}